{
  "gene_name": "Putative transcription factor ovo-like protein 3",
  "term_label": "RNA polymerase II cis-regulatory region sequence-specific DNA binding",
  "term_id": "GO:0000978",
  "gene": "UniProtKB:O00110",
  "gene_symbol": "OVOL3"
}